{
  "gene_name": "Beta-adrenergic receptor kinase 2",
  "gene": "UniProtKB:P35626",
  "term_label": "G protein-coupled receptor signaling pathway",
  "gene_symbol": "GRK3",
  "term_id": "GO:0007186"
}